{
  "term_label": "cytoplasm",
  "gene_name": "BCAS3 microtubule associated cell migration factor",
  "gene_symbol": "BCAS3",
  "gene": "UniProtKB:Q9H6U6",
  "term_id": "GO:0005737"
}